{
  "gene_symbol": "MAGEB10",
  "gene": "UniProtKB:Q96LZ2",
  "term_label": "nucleus",
  "gene_name": "Melanoma-associated antigen B10",
  "term_id": "GO:0005634"
}